regulation of response to gamma radiation [GO:2001228] (biological process) Sources: GOC:obol Subtypes: regulation of cellular response to gamma radiation [GO:1905843], GO:2001229, GO:2001230 Also known as: regulation of response to gamma ray, regulation of response to gamma-ray photon Relationships: is a type of regulation of response to stimulus [GO:0048583]; regulates GO:0010332 Definition: Any process that modulates the frequency, rate or extent of response to gamma radiation.